{
  "gene_symbol": "GRIK4",
  "gene_name": "Glutamate receptor ionotropic, kainate 4",
  "term_id": "GO:0005886",
  "gene": "UniProtKB:Q16099",
  "term_label": "plasma membrane"
}